{
  "gene_name": "Small ribosomal subunit protein eS10",
  "gene_symbol": "RPS10",
  "term_id": "GO:0022627",
  "gene": "UniProtKB:P46783",
  "term_label": "cytosolic small ribosomal subunit"
}